{
  "gene_symbol": "PTGER2",
  "gene": "UniProtKB:P43116",
  "term_label": "adenylate cyclase-activating G protein-coupled receptor signaling pathway",
  "term_id": "GO:0007189",
  "gene_name": "Prostaglandin E2 receptor EP2 subtype"
}